{
  "gene_name": "Adenylate kinase 2, mitochondrial",
  "gene": "UniProtKB:P54819",
  "term_id": "GO:0006172",
  "term_label": "ADP biosynthetic process",
  "gene_symbol": "AK2"
}